{
  "term_label": "sensory perception of sound",
  "term_id": "GO:0007605",
  "gene": "UniProtKB:Q2WEN9",
  "gene_symbol": "CEACAM16",
  "gene_name": "Carcinoembryonic antigen-related cell adhesion molecule 16"
}